{
  "gene": "UniProtKB:Q9UGJ0",
  "term_label": "cytoplasm",
  "term_id": "GO:0005737",
  "gene_name": "5'-AMP-activated protein kinase subunit gamma-2",
  "gene_symbol": "PRKAG2"
}